MIT domain binding [GO:0090541] (molecular function) Definition: Binding to a MIT protein domain. The MIT domain is found in vacuolar sorting proteins, spastin (probable ATPase involved in the assembly or function of nuclear protein complexes), and a sorting nexin, which may play a role in intracellular trafficking. Relationships: is a type of protein domain specific binding [GO:0019904] Sources: GOC:pm, InterPro:IPR007330